{
  "gene": "UniProtKB:Q86UW2",
  "term_id": "GO:0015721",
  "gene_name": "Organic solute transporter subunit beta",
  "term_label": "bile acid and bile salt transport",
  "gene_symbol": "SLC51B"
}